positive regulation of anaphase-promoting complex-dependent catabolic process [GO:1905786] (BP) Relationships: is a type of positive regulation of proteasomal ubiquitin-dependent protein catabolic process [GO:0032436]; is a type of regulation of anaphase-promoting complex-dependent catabolic process [GO:1905784]; positively regulates anaphase-promoting complex-dependent catabolic process [GO:0031145] References: PMID:10921876 Sources: GOC:TermGenie, GO_REF:0000058 Definition: Any process that activates or increases the frequency, rate or extent of anaphase-promoting complex-dependent catabolic process.